regulation of type 2 immune response [GO:0002828] (biological process) Subtypes: negative regulation of type 2 immune response [GO:0002829], GO:0002830, regulation of T-helper 2 cell differentiation [GO:0045628], regulation of T-helper 2 cell cytokine production [GO:2000551] Relationships: is a type of GO:0050776; regulates type 2 immune response [GO:0042092] Sources: GOC:add Also known as: regulation of T-helper 2 type immune response, regulation of Th2 immune response Definition: Any process that modulates the frequency, rate, or extent of a type 2 immune response.